{
  "gene": "UniProtKB:Q9UNZ2",
  "gene_symbol": "NSFL1C",
  "term_label": "cytosol",
  "term_id": "GO:0005829",
  "gene_name": "NSFL1 cofactor p47"
}